{
  "gene": "UniProtKB:Q6PJE2",
  "term_label": "Unknown biological process",
  "gene_symbol": "POMZP3",
  "term_id": "UNKNOWN:0002",
  "gene_name": "POM121 and ZP3 fusion protein"
}